{
  "term_label": "fatty acid biosynthetic process",
  "term_id": "GO:0006633",
  "gene_name": "Acetyl-CoA carboxylase 2",
  "gene": "UniProtKB:O00763",
  "gene_symbol": "ACACB"
}